{
  "gene_name": "Insulin-like growth factor II",
  "gene_symbol": "IGF2",
  "term_label": "growth factor activity",
  "gene": "UniProtKB:P01344",
  "term_id": "GO:0008083"
}